{
  "gene_symbol": "ZNF626",
  "term_label": "RNA polymerase II cis-regulatory region sequence-specific DNA binding",
  "term_id": "GO:0000978",
  "gene_name": "Zinc finger protein 626",
  "gene": "UniProtKB:Q68DY1"
}